{
  "gene_name": "Regulator of G-protein signaling 14",
  "gene_symbol": "RGS14",
  "gene": "UniProtKB:O43566",
  "term_label": "long-term memory",
  "term_id": "GO:0007616"
}